{
  "gene_name": "Receptor-transporting protein 1",
  "gene": "UniProtKB:P59025",
  "term_label": "detection of chemical stimulus involved in sensory perception of bitter taste",
  "term_id": "GO:0001580",
  "gene_symbol": "RTP1"
}